{
  "gene_name": "Zinc transporter ZIP10",
  "gene": "UniProtKB:Q9ULF5",
  "term_label": "zinc ion transmembrane transporter activity",
  "term_id": "GO:0005385",
  "gene_symbol": "SLC39A10"
}